{
  "term_id": "UNKNOWN:0001",
  "term_label": "Unknown molecular function",
  "gene": "UniProtKB:P03979",
  "gene_name": "T cell receptor gamma variable 3",
  "gene_symbol": "TRGV3"
}